{
  "gene": "UniProtKB:O43707",
  "gene_name": "Alpha-actinin-4",
  "gene_symbol": "ACTN4",
  "term_id": "GO:0030864",
  "term_label": "cortical actin cytoskeleton"
}